{
  "gene_name": "Putative uncharacterized protein ANP32CP",
  "term_label": "histone binding",
  "term_id": "GO:0042393",
  "gene": "UniProtKB:O43423",
  "gene_symbol": "ANP32CP"
}